{
  "term_label": "adherens junction organization",
  "gene": "UniProtKB:Q13634",
  "gene_name": "Cadherin-18",
  "gene_symbol": "CDH18",
  "term_id": "GO:0034332"
}